nucleosome binding [GO:0031491] (molecular function) Sources: GOC:mah Subtypes: GO:0031492, GO:0097030 Definition: Binding to a nucleosome, a complex comprised of DNA wound around a multisubunit core and associated proteins, which forms the primary packing unit of DNA into higher order structures. Relationships: is a type of chromatin binding [GO:0003682]; is a type of protein-containing complex binding [GO:0044877]